{
  "term_id": "UNKNOWN:0002",
  "gene_symbol": "NDUFC1",
  "term_label": "Unknown biological process",
  "gene": "UniProtKB:O43677",
  "gene_name": "NADH dehydrogenase [ubiquinone] 1 subunit C1, mitochondrial"
}